negative regulation of determination of dorsal identity [GO:2000016] (biological process) Also known as: negative regulation of determination of adaxial identity Sources: GOC:BHF, GOC:obol Relationships: is a type of negative regulation of multicellular organismal process [GO:0051241]; is a type of regulation of determination of dorsal identity [GO:2000015]; negatively regulates determination of dorsal identity [GO:0048263] Definition: Any process that stops, prevents, or reduces the frequency, rate or extent of determination of dorsal identity.